{
  "gene": "UniProtKB:Q6P4Q7",
  "gene_name": "Metal transporter CNNM4",
  "gene_symbol": "CNNM4",
  "term_label": "magnesium ion transmembrane transporter activity",
  "term_id": "GO:0015095"
}